cell migration involved in sprouting angiogenesis [GO:0002042] (biological process) Regulation: regulated by GO:0090049; positively regulated by GO:0090050; negatively regulated by negative regulation of cell migration involved in sprouting angiogenesis [GO:0090051] References: PMID:16391003 Relationships: is a type of blood vessel endothelial cell migration [GO:0043534]; BFO_0000050 sprouting angiogenesis [GO:0002040] Definition: The orderly movement of endothelial cells into the extracellular matrix in order to form new blood vessels involved in sprouting angiogenesis.